interleukin-17A-mediated signaling pathway [GO:0038173] (biological process) Definition: The series of molecular signals initiated by interleukin-17A binding to its receptor on the surface of a target cell, and ending with the regulation of a downstream cellular process, e.g. transcription. Also known as: IL-17A-mediated signaling pathway, IL17A signaling pathway, interleukin-17A-mediated signalling pathway, interleukin-17A signaling pathway Sources: GOC:jc, GOC:signaling Relationships: is a type of cytokine-mediated signaling pathway [GO:0019221]